{
  "gene": "UniProtKB:A6NHP3",
  "gene_symbol": "SPDYE2B",
  "term_label": "Unknown cellular component",
  "term_id": "UNKNOWN:0003",
  "gene_name": "Speedy protein E2B"
}